{
  "term_id": "GO:0000981",
  "gene_name": "Putative zinc finger protein 705G",
  "gene_symbol": "ZNF705G",
  "gene": "UniProtKB:A8MUZ8",
  "term_label": "DNA-binding transcription factor activity, RNA polymerase II-specific"
}